{
  "gene_symbol": "C6orf141",
  "gene": "UniProtKB:Q5SZD1",
  "term_id": "UNKNOWN:0002",
  "gene_name": "Uncharacterized protein C6orf141",
  "term_label": "Unknown biological process"
}